nuclear replication fork [GO:0043596] (cellular component) Sources: GOC:jl, GOC:mtg_sensu Definition: The Y-shaped region of a nuclear replicating DNA molecule, resulting from the separation of the DNA strands and in which the synthesis of new strands takes place. Also includes associated protein complexes. Relationships: is a type of replication fork [GO:0005657]; is part of nuclear chromosome [GO:0000228]; has part CMG complex [GO:0071162]